protein catenane formation [GO:0018419] (biological process) Definition: The aggregation, arrangement and bonding together of a protein structure comprising two or more rings that are interlocked but not covalently joined; resembling the links of a chain. Relationships: is a type of GO:0065003 Sources: ISBN:0198506732